{
  "term_id": "GO:0016082",
  "term_label": "synaptic vesicle priming",
  "gene": "UniProtKB:Q9UJD0",
  "gene_symbol": "RIMS3",
  "gene_name": "Regulating synaptic membrane exocytosis protein 3"
}